negative regulation of synaptic vesicle membrane organization [GO:1901633] (biological process) Definition: Any process that stops, prevents or reduces the frequency, rate or extent of synaptic vesicle membrane organization. Subtypes: negative regulation of synaptic vesicle fusion to presynaptic active zone membrane [GO:0031631] Also known as: down regulation of synaptic vesicle membrane organisation, down regulation of synaptic vesicle membrane organization, down-regulation of synaptic vesicle membrane organisation, down-regulation of synaptic vesicle membrane organization, downregulation of synaptic vesicle membrane organisation, downregulation of synaptic vesicle membrane organization, negative regulation of synaptic vesicle membrane organisation, down regulation of SLMV biogenesis, down-regulation of SLMV biogenesis, downregulation of SLMV biogenesis, inhibition of SLMV biogenesis, inhibition of synaptic vesicle membrane organisation, inhibition of synaptic vesicle membrane organization, inhibition of synaptic vesicle membrane organization and biogenesis, negative regulation of SLMV biogenesis, down regulation of synaptic vesicle membrane organization and biogenesis, down-regulation of synaptic vesicle membrane organization and biogenesis, downregulation of synaptic vesicle membrane organization and biogenesis, negative regulation of synaptic vesicle membrane organization and biogenesis Relationships: is a type of negative regulation of cellular component organization [GO:0051129]; is a type of regulation of synaptic vesicle membrane organization [GO:1901632]; negatively regulates synaptic vesicle membrane organization [GO:0048499] References: PMID:22426000 Sources: GOC:TermGenie